{
  "gene": "UniProtKB:Q96QF0",
  "gene_symbol": "RAB3IP",
  "term_label": "guanyl-nucleotide exchange factor activity",
  "gene_name": "Rab-3A-interacting protein",
  "term_id": "GO:0005085"
}